{
  "gene": "UniProtKB:O75907",
  "term_id": "GO:0004144",
  "gene_name": "Diacylglycerol O-acyltransferase 1",
  "term_label": "diacylglycerol O-acyltransferase activity",
  "gene_symbol": "DGAT1"
}